structural constituent of carboxysome shell [GO:0043886] (molecular function) References: PMID:28934381 Sources: GOC:jl Definition: The action of a molecule that contributes to the structural integrity of a carboxysome shell, an organelle found in all cyanobacteria and some chemoautotrophs, consisting of a proteinaceous coat and enzymes for the fixation of CO2. Also known as: structural constituent of carboxysome Relationships: is a type of structural molecule activity [GO:0005198]; occurs in GO:0031470